{
  "term_label": "Unknown biological process",
  "gene": "UniProtKB:Q8NFZ3",
  "gene_symbol": "NLGN4Y",
  "term_id": "UNKNOWN:0002",
  "gene_name": "Neuroligin-4, Y-linked"
}